{
  "gene_symbol": "ACP4",
  "term_label": "protein tyrosine phosphatase activity",
  "gene": "UniProtKB:Q9BZG2",
  "gene_name": "Testicular acid phosphatase",
  "term_id": "GO:0004725"
}